sieve cell differentiation [GO:0048756] (BP) Definition: The process in which a relatively unspecialized cell acquires specialized features of a sieve cell. A sieve cell is a type of sieve element that has relatively undifferentiated sieve areas (with narrow pores). The sieve areas are rather uniform in structure on all walls; that is, there are no sieve plates. Typical of gymnosperms and lower vascular plants. The sieve element is the cell in the phloem tissue concerned with mainly longitudinal conduction of food materials. Sources: GOC:jid, PO:0025415, POC:curators Relationships: is a type of sieve element differentiation [GO:0090603]; is part of GO:0010088